{
  "term_label": "structural constituent of ribosome",
  "gene": "UniProtKB:P62829",
  "gene_symbol": "RPL23",
  "gene_name": "Large ribosomal subunit protein uL14",
  "term_id": "GO:0003735"
}